{
  "gene": "UniProtKB:Q13621",
  "term_id": "GO:0055078",
  "gene_name": "Solute carrier family 12 member 1",
  "term_label": "sodium ion homeostasis",
  "gene_symbol": "SLC12A1"
}